positive regulation of DNA replication initiation [GO:1903468] (BP) Definition: Any process that activates or increases the frequency, rate or extent of DNA replication initiation involved in mitotic DNA replication. Relationships: is a type of GO:0032298; is_a GO:1903465; is_a regulation of mitotic DNA replication initiation [GO:1903466]; positively regulates GO:1902975 Also known as: positive regulation of DNA replication initiation involved in mitotic cell cycle DNA replication, up regulation of DNA replication initiation involved in mitotic DNA replication, up regulation of DNA replication initiation involved in mitotic cell cycle DNA replication, up-regulation of DNA replication initiation involved in mitotic DNA replication, up-regulation of DNA replication initiation involved in mitotic cell cycle DNA replication, upregulation of DNA replication initiation involved in mitotic DNA replication, upregulation of DNA replication initiation involved in mitotic cell cycle DNA replication, activation of DNA replication initiation involved in mitotic DNA replication, activation of DNA replication initiation involved in mitotic cell cycle DNA replication References: PMID:1234 Sources: GOC:TermGenie, GOC:mtg_cell_cycle, GO_REF:0000058